retrograde neuronal dense core vesicle transport [GO:1990049] (biological process) References: PMID:23358451, PMID:24762653 Sources: GOC:kmv Also known as: retrograde dense core granule trafficking, retrograde dense core granule transport Definition: The directed movement of neuronal dense core vesicles along axonal microtubules towards the cell body. Regulation: regulated by GO:1901954; RO_0002212 by negative regulation of retrograde dense core granule transport [GO:1901955]; positively regulated by positive regulation of retrograde dense core granule transport [GO:1901956] Relationships: is a type of retrograde axonal transport [GO:0008090]; is a type of GO:0047496; is a type of GO:0099519